{
  "term_id": "GO:0006487",
  "gene_symbol": "MGAT4C",
  "gene": "UniProtKB:Q9UBM8",
  "gene_name": "Alpha-1,3-mannosyl-glycoprotein 4-beta-N-acetylglucosaminyltransferase C",
  "term_label": "protein N-linked glycosylation"
}